{
  "gene": "UniProtKB:P13521",
  "term_label": "extracellular space",
  "gene_symbol": "SCG2",
  "gene_name": "Secretogranin-2",
  "term_id": "GO:0005615"
}